{
  "term_id": "GO:0070475",
  "gene": "UniProtKB:P46087",
  "gene_symbol": "NOP2",
  "term_label": "rRNA base methylation",
  "gene_name": "Probable 28S rRNA (cytosine(4447)-C(5))-methyltransferase"
}